{
  "term_label": "protein kinase C binding",
  "gene_name": "Sequestosome-1",
  "gene": "UniProtKB:Q13501",
  "gene_symbol": "SQSTM1",
  "term_id": "GO:0005080"
}